{
  "gene": "UniProtKB:Q99687",
  "term_label": "eye development",
  "term_id": "GO:0001654",
  "gene_symbol": "MEIS3",
  "gene_name": "Homeobox protein Meis3"
}